{
  "term_label": "plasma membrane",
  "term_id": "GO:0005886",
  "gene_symbol": "SLC28A1",
  "gene": "UniProtKB:O00337",
  "gene_name": "Sodium_nucleoside cotransporter 1"
}